kinase regulator activity [GO:0019207] (molecular function) Subtypes: acetylglutamate kinase regulator activity [GO:0010307], kinase activator activity [GO:0019209], kinase inhibitor activity [GO:0019210], protein kinase regulator activity [GO:0019887], phosphatidylinositol 3-kinase regulator activity [GO:0035014], 1-phosphatidylinositol-3-kinase regulator activity [GO:0046935] Sources: GOC:ai Relationships: is a type of enzyme regulator activity [GO:0030234]; regulates kinase activity [GO:0016301] Definition: Modulates the activity of a kinase, an enzyme which catalyzes of the transfer of a phosphate group, usually from ATP, to a substrate molecule.